{
  "term_id": "UNKNOWN:0001",
  "gene": "UniProtKB:Q9HAU5",
  "gene_symbol": "UPF2",
  "gene_name": "Regulator of nonsense transcripts 2",
  "term_label": "Unknown molecular function"
}